{
  "gene_symbol": "CHTOP",
  "term_label": "nuclear speck",
  "gene": "UniProtKB:Q9Y3Y2",
  "gene_name": "Chromatin target of PRMT1 protein",
  "term_id": "GO:0016607"
}